{
  "term_id": "GO:0003777",
  "gene_name": "Kinesin-like protein KIFC1",
  "gene_symbol": "KIFC1",
  "term_label": "microtubule motor activity",
  "gene": "UniProtKB:Q9BW19"
}